purine nucleotide interconversion [GO:0015950] (biological process) Relationships: is a type of GO:0006163; is a type of nucleobase-containing small molecule interconversion [GO:0015949] Definition: The chemical reactions and pathways by which a purine nucleotide is synthesized from another purine nucleotide. Sources: GOC:mah, ISBN:0306444747, ISBN:0471394831 Subtypes: purine ribonucleotide interconversion [GO:0015951], purine deoxyribonucleotide interconversion [GO:0015952]